{
  "term_label": "Unknown molecular function",
  "gene_symbol": "TRBV5-4",
  "gene": "UniProtKB:A0A0C4DH59",
  "gene_name": "T cell receptor beta variable 5-4",
  "term_id": "UNKNOWN:0001"
}